sulphoglycolysis [GO:0061722] (biological process) Relationships: is a type of GO:0006090; is_a generation of precursor metabolites and energy [GO:0006091]; is a type of ATP metabolic process [GO:0046034]; is a type of GO:0046496; is a type of 6-sulfoquinovose(1-) catabolic process [GO:1902777]; has part glyceraldehyde-3-phosphate dehydrogenase (NAD+) (phosphorylating) activity [GO:0004365]; has part phosphoglycerate kinase activity [GO:0004618]; has part phosphoglycerate mutase activity [GO:0004619]; has part GO:0004634; has part pyruvate kinase activity [GO:0004743]; has part triose-phosphate isomerase activity [GO:0004807]; has part GO:0061720 Definition: The chemical reactions and pathways resulting in the breakdown of 6-sulfoquinovose(1-) resulting in the formation of glycerone phosphate (DHAP) and pyruvate. Also known as: sulfoglycolysis References: PMID:24463506 Sources: GOC:dph